{
  "term_label": "plasma membrane",
  "gene_symbol": "OR4Q3",
  "term_id": "GO:0005886",
  "gene": "UniProtKB:Q8NH05",
  "gene_name": "Olfactory receptor 4Q3"
}